sulfate ion homeostasis [GO:0055063] (biological process) Definition: Any process involved in the maintenance of an internal steady state of sulfate ions within an organism or cell. Sources: GOC:jid, GOC:mah Also known as: sulfate homeostasis, sulphate ion homeostasis Relationships: is a type of inorganic ion homeostasis [GO:0098771] Subtypes: intracellular sulfate ion homeostasis [GO:0030642]